{
  "term_id": "GO:1902531",
  "gene": "UniProtKB:P21359",
  "gene_name": "Neurofibromin",
  "gene_symbol": "NF1",
  "term_label": "regulation of intracellular signal transduction"
}